{
  "term_id": "GO:0000386",
  "gene_symbol": "SLU7",
  "gene": "UniProtKB:O95391",
  "term_label": "second spliceosomal transesterification activity",
  "gene_name": "Pre-mRNA-splicing factor SLU7"
}